{
  "term_id": "GO:0000381",
  "gene_symbol": "RBM15B",
  "gene_name": "Putative RNA-binding protein 15B",
  "term_label": "regulation of alternative mRNA splicing, via spliceosome",
  "gene": "UniProtKB:Q8NDT2"
}